histone H2AQ104 methyltransferase activity [GO:1990259] (molecular function) Definition: Catalysis of the reaction: L-glutamine(104)-[histone H2A] + S-adenosyl-L-methionine = N(5)-methyl-L-glutamine(104)-[histone H2A] + S-adenosyl-L-homocysteine + H+. Note that this corresponds to Q105 in yeast. Relationships: is a type of protein-glutamine N-methyltransferase activity [GO:0036009]; is a type of GO:0140940 Note: Note that the residue position corresponds to the canonical human H2A2A histone (UniProtKB:Q6FI13); this residue is conserved across all eukaryotes. Note that this resudue is missing from the H2AZ clade. Residue 1 is the first residue following removal of the initiating Methionine (Met). Note that each histone is encoded by multiple genes, and sequences may vary across different genes within an organism. References: PMID:24352239 Sources: RHEA:43228 Also known as: histone glutamine N-methyltransferase activity, histone glutamine methylase activity, histone glutamine methyltransferase activity, histone-glutamine N-methyltransferase activity, histone-glutamine methyltransferase activity